{
  "term_id": "GO:0003723",
  "term_label": "RNA binding",
  "gene_symbol": "DICER1",
  "gene_name": "Endoribonuclease Dicer",
  "gene": "UniProtKB:Q9UPY3"
}